U2-type post-spliceosomal complex [GO:0071021] (CC) Relationships: is a type of U2-type spliceosomal complex [GO:0005684]; is a type of post-spliceosomal complex [GO:0071020]; BFO_0000051 U2 snRNP [GO:0005686]; has part U6 snRNP [GO:0005688] Also known as: major post-spliceosomal complex, GT-AG post-spliceosomal complex, mammalian U2-type spliceosomal complex C2, yeast U2-type spliceosomal complex A2-3 Definition: A spliceosomal complex that is formed following the second splicing event and contains the spliced product, the excised intron, and three snRNPs, U5, U2 and U6. Sources: GOC:krc, GOC:mah, ISBN:0879695897, ISBN:0879697393